symmetric stem cell division [GO:0098724] (biological process) Note: Examples include the self-renewal of spermatogonial stem cells and (some) division during amplification of skeletal muscle satellite cell populations. References: PMID:19948499, PMID:23303905 Relationships: is a type of GO:0017145; is a type of GO:0098725 Subtypes: symmetric division of skeletal muscle satellite stem cell [GO:0098726], germline stem cell symmetric division [GO:0098729] Definition: Symmetric division of a stem cell to produce two stem cells of the same type as the parent. Symmetric stem cell division is necessary for amplification of stem cell populations in the absence of sources of stem cells external to an existing population.